{
  "term_id": "GO:0043025",
  "term_label": "neuronal cell body",
  "gene_name": "Double-stranded RNA-binding protein Staufen homolog 2",
  "gene": "UniProtKB:Q9NUL3",
  "gene_symbol": "STAU2"
}